right lateral basal body pair [GO:0097564] (CC) Definition: Set of two basal bodies found in Giardia species (trophozoite stage). It comprises the anterior and ventral basal bodies located to the left of the right nucleus of the trophozoite when viewed dorsally. References: PMID:16607022, PMID:5961344 Sources: GOC:giardia, ISBN:9780124260207 Relationships: is a type of cellular anatomical structure [GO:0110165]; is part of cell projection [GO:0042995]; has part right anterior basal body [GO:1902672]; has part right ventral basal body [GO:1902676] Note: Due to the asymmetric nature of the Giardia trophozoite, this term is defined spatially as the trophozoite is viewed from the dorsal side, with the two nuclei dorsal to the ventral disc, and the ventral disc toward the anterior.